{
  "gene": "UniProtKB:Q03721",
  "term_label": "dendrite membrane",
  "term_id": "GO:0032590",
  "gene_name": "Potassium voltage-gated channel subfamily C member 4",
  "gene_symbol": "KCNC4"
}